{
  "term_label": "animal organ morphogenesis",
  "gene": "UniProtKB:Q9C0F0",
  "gene_name": "Putative Polycomb group protein ASXL3",
  "gene_symbol": "ASXL3",
  "term_id": "GO:0009887"
}